{
  "term_id": "GO:0003743",
  "gene": "UniProtKB:P05198",
  "term_label": "translation initiation factor activity",
  "gene_symbol": "EIF2S1",
  "gene_name": "Eukaryotic translation initiation factor 2 subunit 1"
}